positive regulation of G protein-coupled receptor signaling pathway [GO:0045745] (biological process) Sources: GOC:go_curators Relationships: is a type of regulation of G protein-coupled receptor signaling pathway [GO:0008277]; is a type of positive regulation of signal transduction [GO:0009967]; positively regulates G protein-coupled receptor signaling pathway [GO:0007186] Also known as: positive regulation of G protein coupled receptor protein signaling pathway, positive regulation of G protein coupled receptor protein signalling pathway, positive regulation of G-protein coupled receptor protein signaling pathway, positive regulation of G-protein coupled receptor protein signalling pathway, positive regulation of G-protein-coupled receptor protein signaling pathway, positive regulation of G-protein-coupled receptor protein signalling pathway, positive regulation of GPCR protein signaling pathway, positive regulation of GPCR protein signalling pathway, up regulation of G-protein coupled receptor protein signaling pathway, up-regulation of G-protein coupled receptor protein signaling pathway, upregulation of G-protein coupled receptor protein signaling pathway, activation of G-protein coupled receptor protein signaling pathway, stimulation of G-protein coupled receptor protein signaling pathway Definition: Any process that activates or increases the frequency, rate or extent of G protein-coupled receptor signaling pathway activity. Subtypes: positive regulation of dopamine receptor signaling pathway [GO:0060161], positive regulation of adenosine receptor signaling pathway [GO:0060168], positive regulation of chemokine-mediated signaling pathway [GO:0070101], positive regulation of thrombin-activated receptor signaling pathway [GO:0070496], positive regulation of adenylate cyclase-activating adrenergic receptor signaling pathway [GO:0071879], GO:0106071, positive regulation of angiotensin-activated signaling pathway [GO:0110063], positive regulation of phospholipase C-activating G protein-coupled receptor signaling pathway [GO:1900738], negative regulation of inhibitory G protein-coupled receptor phosphorylation [GO:1904324], GO:2000127, positive regulation of opioid receptor signaling pathway [GO:2000476]